NADPH regeneration [GO:0006740] (biological process) Sources: GOC:mah Definition: A metabolic process that generates a pool of NADPH by the reduction of NADP+. Subtypes: pentose-phosphate shunt [GO:0006098], GO:0009051, GO:0009780 Also known as: NADP (reduced) regeneration, reduced NADP regeneration, reduced nicotinamide adenine dinucleotide phosphate regeneration Relationships: is_a generation of precursor metabolites and energy [GO:0006091]; is a type of NADP+ metabolic process [GO:0006739]